{
  "gene": "UniProtKB:Q99536",
  "gene_name": "Synaptic vesicle membrane protein VAT-1 homolog",
  "gene_symbol": "VAT1",
  "term_label": "negative regulation of mitochondrial fusion",
  "term_id": "GO:0010637"
}